{
  "gene_symbol": "CHRNA5",
  "term_id": "GO:0007271",
  "gene_name": "Neuronal acetylcholine receptor subunit alpha-5",
  "gene": "UniProtKB:P30532",
  "term_label": "synaptic transmission, cholinergic"
}